{
  "gene": "UniProtKB:Q9NQW8",
  "term_label": "photoreceptor outer segment",
  "term_id": "GO:0001750",
  "gene_name": "Cyclic nucleotide-gated cation channel beta-3",
  "gene_symbol": "CNGB3"
}